{
  "gene_symbol": "BAIAP2L1",
  "term_label": "Unknown molecular function",
  "term_id": "UNKNOWN:0001",
  "gene_name": "Brain-specific angiogenesis inhibitor 1-associated protein 2-like protein 1",
  "gene": "UniProtKB:Q9UHR4"
}